{
  "term_label": "beta-catenin binding",
  "gene": "UniProtKB:P55289",
  "gene_symbol": "CDH12",
  "gene_name": "Cadherin-12",
  "term_id": "GO:0008013"
}